{
  "gene_symbol": "CDHR1",
  "term_id": "GO:0005886",
  "term_label": "plasma membrane",
  "gene": "UniProtKB:Q96JP9",
  "gene_name": "Cadherin-related family member 1"
}